phosphatidylinositol-4,5-bisphosphate 5-phosphatase activity [GO:0004439] (molecular function) Relationships: is a type of phosphatidylinositol phosphate 5-phosphatase activity [GO:0034595]; is_a GO:0106019 Also known as: phosphatidylinositol 4,5-bisphosphate phosphatase activity, phosphatidylinositol-bisphosphatase activity, triphosphoinositide phosphatase activity, triphosphoinositide phosphomonoesterase activity, PI(4,5)P2 5-phosphatase activity, PtdIns(4,5)P(2) 5-phosphatase activity, PtdIns(4,5)P2 5-phosphatase activity, phosphatidyl-myo-inositol-4,5-bisphosphate phosphatase activity Sources: RHEA:22764 Definition: Catalysis of the reaction: 1-phosphatidyl-1D-myo-inositol 4,5-bisphosphate + H2O = 1-phosphatidyl-1D-myo-inositol 4-phosphate + phosphate.